rod photoreceptor disc membrane [GO:0120202] (cellular component) References: PMID:19501669, PMID:26574505, PMID:6771304 Sources: GOC:krc, GOC:pde Definition: Stack of disc membranes located inside a rod photoreceptor outer segment, and containing densely packed molecules of rhodopsin photoreceptor proteins that traverse the lipid bilayer. It is thought that rod disc membranes arise as evaginations of the ciliary membrane near the base of the outer segment, which then become completely separated from the ciliary membrane, during the development of the rod outer segment. Relationships: is a type of cytoplasmic vesicle membrane [GO:0030659]; is a type of photoreceptor disc membrane [GO:0097381]